{
  "gene": "UniProtKB:Q96NE9",
  "gene_symbol": "FRMD6",
  "term_label": "protein sequestering activity",
  "gene_name": "FERM domain-containing protein 6",
  "term_id": "GO:0140311"
}